cleavage furrow rim [GO:0090688] (cellular component) References: PMID:27082518 Sources: GOC:vw Definition: The part of the cleavage furrow closest to the cell surface. Relationships: is a type of cellular anatomical structure [GO:0110165]; is part of cleavage furrow [GO:0032154]